{
  "term_label": "small-subunit processome",
  "gene_symbol": "HEATR1",
  "gene_name": "HEAT repeat-containing protein 1",
  "term_id": "GO:0032040",
  "gene": "UniProtKB:Q9H583"
}